interleukin-18 production [GO:0032621] (biological process) Definition: The appearance of interleukin-18 due to biosynthesis or secretion following a cellular stimulus, resulting in an increase in its intracellular or extracellular levels. Also known as: IGIF production, IL-18 production, IL1F4 production, interleukin-18 biosynthetic process, interleukin-18 secretion Sources: GOC:mah Relationships: is a type of GO:0001816 Regulation: RO_0002211 by regulation of interleukin-18 production [GO:0032661]; negatively regulated by GO:0032701; RO_0002213 by positive regulation of interleukin-18 production [GO:0032741]